chloroplast [GO:0009507] (cellular component) Definition: A chlorophyll-containing plastid with thylakoids organized into grana and frets, or stroma thylakoids, and embedded in a stroma. Sources: ISBN:0471245208 Relationships: is a type of plastid [GO:0009536]